positive regulation of odontogenesis of dentin-containing tooth [GO:0042488] (biological process) Also known as: activation of odontogenesis, stimulation of odontogenesis, up regulation of odontogenesis, up-regulation of odontogenesis, upregulation of odontogenesis, positive regulation of odontogenesis of dentine-containing teeth, positive regulation of odontogenesis of dentine-containing tooth Subtypes: positive regulation of dentin-containing tooth bud formation by mesenchymal-epithelial signaling [GO:0060640] Definition: Any process that activates or increases the frequency, rate or extent of the formation and development of teeth, the hard, bony appendages that are borne on the jaws, or on other bones in the walls of the mouth or pharynx of most vertebrates. Relationships: is a type of GO:0042482; is a type of regulation of odontogenesis of dentin-containing tooth [GO:0042487]; positively regulates GO:0042475 References: PMID:15355794 Sources: GOC:jl